{
  "gene_symbol": "STK33",
  "gene_name": "Serine_threonine-protein kinase 33",
  "gene": "UniProtKB:Q9BYT3",
  "term_label": "protein serine/threonine kinase activity",
  "term_id": "GO:0004674"
}